{
  "term_id": "GO:0005085",
  "term_label": "guanyl-nucleotide exchange factor activity",
  "gene_name": "Rho guanine nucleotide exchange factor 5",
  "gene": "UniProtKB:Q12774",
  "gene_symbol": "ARHGEF5"
}